{
  "gene_name": "Protein ZNF365",
  "term_id": "GO:0010569",
  "gene_symbol": "ZNF365",
  "term_label": "regulation of double-strand break repair via homologous recombination",
  "gene": "UniProtKB:Q70YC5"
}